{
  "gene_name": "Methyl-CpG-binding protein 2",
  "term_label": "double-stranded methylated DNA binding",
  "gene": "UniProtKB:P51608",
  "term_id": "GO:0010385",
  "gene_symbol": "MECP2"
}